{
  "term_id": "GO:0031410",
  "gene": "UniProtKB:Q96PP8",
  "gene_name": "Guanylate-binding protein 5",
  "gene_symbol": "GBP5",
  "term_label": "cytoplasmic vesicle"
}